{
  "term_label": "response to exogenous dsRNA",
  "gene_symbol": "IFNA1",
  "term_id": "GO:0043330",
  "gene": "UniProtKB:P01562",
  "gene_name": "Interferon alpha-1_13"
}